G protein-coupled receptor complex [GO:0097648] (CC) Sources: GOC:bhm Definition: A protein complex that contains G protein-coupled receptors. Subtypes: G protein-coupled receptor dimeric complex [GO:0038037], calcitonin family receptor complex [GO:1903439] Also known as: G-protein coupled receptor complex Relationships: is a type of plasma membrane signaling receptor complex [GO:0098802]